{
  "gene_symbol": "TTC29",
  "gene_name": "Tetratricopeptide repeat protein 29",
  "term_id": "GO:0003341",
  "term_label": "cilium movement",
  "gene": "UniProtKB:Q8NA56"
}